neuronal cell body [GO:0043025] (cellular component) Definition: The portion of a neuron that includes the nucleus, but excludes cell projections such as axons and dendrites. Sources: GOC:go_curators Also known as: neuron cell body, neuronal cell soma Note: Note that 'cell body' and 'cell soma' are not used in the literature for cells that lack projections, nor for some cells (e.g. yeast with mating projections) that do have projections. Relationships: is a type of cell body [GO:0044297]; is part of somatodendritic compartment [GO:0036477]